{
  "term_label": "clathrin-coated vesicle",
  "gene_symbol": "HIP1",
  "term_id": "GO:0030136",
  "gene_name": "Huntingtin-interacting protein 1",
  "gene": "UniProtKB:O00291"
}